{
  "term_label": "odorant binding",
  "gene_symbol": "OR5W2",
  "gene": "UniProtKB:Q8NH69",
  "term_id": "GO:0005549",
  "gene_name": "Olfactory receptor 5W2"
}